{
  "gene": "UniProtKB:Q9UMR3",
  "term_id": "GO:0000981",
  "term_label": "DNA-binding transcription factor activity, RNA polymerase II-specific",
  "gene_name": "T-box transcription factor TBX20",
  "gene_symbol": "TBX20"
}